ventral spinal cord development [GO:0021517] (biological process) Sources: GOC:cls, GOC:dgh, GOC:dph, GOC:jid, GO_REF:0000021 Definition: The process whose specific outcome is the progression of the ventral region of the spinal cord over time, from its formation to the mature structure. The neurons of the ventral region of the mature spinal cord participate in motor output. Relationships: is a type of anatomical structure development [GO:0048856]; is part of spinal cord development [GO:0021510]